{
  "term_id": "UNKNOWN:0001",
  "gene_symbol": "ERCC6L2-AS1",
  "gene": "UniProtKB:Q8WZB0",
  "gene_name": "Putative uncharacterized protein ERCC6L2-AS1",
  "term_label": "Unknown molecular function"
}